morphogenesis of a polarized epithelium [GO:0001738] (biological process) Also known as: epithelial polarization Relationships: is a type of morphogenesis of an epithelium [GO:0002009] Definition: The morphogenetic process in which the anatomical structures of a polarized epithelium are generated and organized. A polarized epithelium is an epithelium where the epithelial sheet is oriented with respect to the planar axis. Sources: GOC:dph